{
  "gene_name": "Ribosomal RNA small subunit methyltransferase NEP1",
  "term_id": "GO:0070475",
  "gene_symbol": "EMG1",
  "term_label": "rRNA base methylation",
  "gene": "UniProtKB:Q92979"
}